{
  "gene_symbol": "TCF23",
  "term_id": "UNKNOWN:0003",
  "gene": "UniProtKB:Q7RTU1",
  "gene_name": "Transcription factor 23",
  "term_label": "Unknown cellular component"
}